{
  "gene_symbol": "PITX2",
  "gene": "UniProtKB:Q99697",
  "term_label": "regulation of transcription by RNA polymerase II",
  "term_id": "GO:0006357",
  "gene_name": "Pituitary homeobox 2"
}